arabinogalactan protein metabolic process [GO:0010405] (biological process) Relationships: is a type of cell wall proteoglycan metabolic process [GO:0010384] Also known as: arabinogalactan protein metabolism Definition: The chemical reactions and pathways involving a cell wall arabinogalactan II glycoprotein, which is composed of a group of core protein of highly varying length and domain complexity. These are O-glycosylated at one or more hydroxyproline residues by arabinogalactan (AG) type II groups, which consist of (1->3)-beta-galactan and (1->6)-beta-linked galactan chains connected to each other by (1->3,1->6)-linked branch points, O-3 and O-6 positions substituted with terminal arabinosyl residues. Also, rhamnose, fucose, glucuronic and galacturonic acid can be present in the glycan structures. Subtypes: GO:0010406, non-classical arabinogalactan protein metabolic process [GO:0010407] Sources: GOC:tair_curators